regulation of nitric oxide biosynthetic process [GO:0045428] (biological process) Subtypes: negative regulation of nitric oxide biosynthetic process [GO:0045019], positive regulation of nitric oxide biosynthetic process [GO:0045429] Relationships: is a type of regulation of biosynthetic process [GO:0009889]; is a type of GO:0080164; regulates nitric oxide biosynthetic process [GO:0006809] Also known as: regulation of nitric oxide anabolism, regulation of nitric oxide biosynthesis, regulation of nitric oxide formation, regulation of nitric oxide synthesis Sources: GOC:go_curators Definition: Any process that modulates the frequency, rate or extent of the chemical reactions and pathways resulting in the formation of nitric oxide.